{
  "gene_name": "Adhesion G protein-coupled receptor A2",
  "term_id": "GO:0090263",
  "gene": "UniProtKB:Q96PE1",
  "gene_symbol": "ADGRA2",
  "term_label": "positive regulation of canonical Wnt signaling pathway"
}